{
  "gene_name": "Transmembrane emp24 domain-containing protein 4",
  "term_label": "endoplasmic reticulum",
  "gene": "UniProtKB:Q7Z7H5",
  "gene_symbol": "TMED4",
  "term_id": "GO:0005783"
}